{
  "term_id": "UNKNOWN:0002",
  "gene": "UniProtKB:P0C7Q2",
  "term_label": "Unknown biological process",
  "gene_name": "Age-related maculopathy susceptibility protein 2",
  "gene_symbol": "ARMS2"
}